inositol 1,4,5-trisphosphate-gated calcium channel activity [GO:0005220] (molecular function) References: PMID:28416699, PMID:8660280 Sources: GOC:mah, GOC:signaling, Wikipedia:Inositol_trisphosphate_receptor Relationships: is_a intracellularly gated calcium channel activity [GO:0015278]; has part inositol 1,4,5 trisphosphate binding [GO:0070679] Also known as: IP3 receptor activity, InsP3 receptor, inositol 1,4,5-trisphosphate-sensitive calcium-release channel activity, inositol-1,4,5-trisphosphate receptor activity Definition: Enables the transmembrane transfer of a calcium ion by a channel that opens when inositol 1,4,5-trisphosphate (IP3) has been bound by the channel complex or one of its constituent parts. Subtypes: GO:0098695